{
  "term_label": "nucleus",
  "gene_name": "Zinc finger protein 439",
  "term_id": "GO:0005634",
  "gene_symbol": "ZNF439",
  "gene": "UniProtKB:Q8NDP4"
}